{
  "term_id": "GO:0099550",
  "gene": "UniProtKB:Q86Z23",
  "gene_name": "Complement C1q-like protein 4",
  "gene_symbol": "C1QL4",
  "term_label": "trans-synaptic signaling, modulating synaptic transmission"
}